NSL complex [GO:0044545] (cellular component) Definition: A histone acetyltransferase complex that catalyzes the acetylation of a histone H4 lysine residues at several positions. In human, it contains the catalytic subunit MOF, NSL1/KIAA1267, NSL2/KANSL2, NSL3/KANSL3, MCRS1, PHF20, OGT1, WDR5 and HCF1. References: PMID:20018852 Sources: GOC:lb Relationships: is a type of H4 histone acetyltransferase complex [GO:1902562] Also known as: non-specific lethal complex